{
  "gene_symbol": "SLC2A8",
  "term_id": "GO:1904659",
  "term_label": "D-glucose transmembrane transport",
  "gene": "UniProtKB:Q9NY64",
  "gene_name": "Solute carrier family 2, facilitated glucose transporter member 8"
}